acetylspermidine deacetylase activity [GO:0047611] (molecular function) Also known as: N-acetylspermidine deacetylase activity, 8-N-acetylspermidine amidohydrolase activity, N(1)-acetylspermidine amidohydrolase activity, N(8)-acetylspermidine amidohydrolase activity, N(8)-acetylspermidine deacetylase activity, N(8)-monoacetylspermidine deacetylase activity, N1-acetylspermidine amidohydrolase activity, N8-acetylspermidine amidohydrolase activity, N8-acetylspermidine deacetylase activity, N8-monoacetylspermidine deacetylase activity Relationships: is a type of hydrolase activity, acting on carbon-nitrogen (but not peptide) bonds, in linear amides [GO:0016811]; is a type of GO:0019213 Definition: Catalysis of the reaction: N(8)-acetylspermidine + H2O = acetate + spermidine. Sources: EC:3.5.1.48, RHEA:23928